{
  "gene_symbol": "RRN3P2",
  "term_label": "RNA polymerase I general transcription initiation factor activity",
  "gene": "UniProtKB:A6NIE6",
  "gene_name": "Putative RRN3-like protein RRN3P2",
  "term_id": "GO:0001181"
}